{
  "gene_name": "Interleukin-6 receptor subunit beta",
  "term_id": "GO:0009897",
  "gene": "UniProtKB:P40189",
  "gene_symbol": "IL6ST",
  "term_label": "external side of plasma membrane"
}